larval somatic muscle development [GO:0007526] (biological process) Relationships: is a type of GO:0007525; is part of GO:0002164 Regulation: regulated by GO:0062229; negatively regulated by negative regulation of larval somatic muscle development [GO:0062230]; positively regulated by positive regulation of larval somatic muscle development [GO:0062231] Definition: The process whose specific outcome is the progression of the larval somatic muscle over time, from its formation to the mature structure. Sources: GOC:jid